{
  "gene_symbol": "BPIFA1",
  "term_label": "extracellular space",
  "gene": "UniProtKB:Q9NP55",
  "term_id": "GO:0005615",
  "gene_name": "BPI fold-containing family A member 1"
}